{
  "term_label": "mitochondrial DNA replication",
  "gene_symbol": "MGME1",
  "gene_name": "Mitochondrial genome maintenance exonuclease 1",
  "gene": "UniProtKB:Q9BQP7",
  "term_id": "GO:0006264"
}